{
  "gene_name": "Arginine_serine-rich coiled-coil protein 2",
  "term_id": "UNKNOWN:0001",
  "term_label": "Unknown molecular function",
  "gene": "UniProtKB:Q7L4I2",
  "gene_symbol": "RSRC2"
}